{
  "gene": "UniProtKB:Q8NHP8",
  "gene_symbol": "PLBD2",
  "term_label": "extracellular region",
  "term_id": "GO:0005576",
  "gene_name": "Putative phospholipase B-like 2"
}